{
  "gene": "UniProtKB:P62487",
  "term_label": "transcription initiation at RNA polymerase II promoter",
  "gene_name": "DNA-directed RNA polymerase II subunit RPB7",
  "gene_symbol": "POLR2G",
  "term_id": "GO:0006367"
}